{
  "gene_symbol": "HOXA4",
  "term_label": "nucleoplasm",
  "term_id": "GO:0005654",
  "gene_name": "Homeobox protein Hox-A4",
  "gene": "UniProtKB:Q00056"
}